{
  "gene_symbol": "KBTBD7",
  "term_label": "ubiquitin-like ligase-substrate adaptor activity",
  "gene_name": "Kelch repeat and BTB domain-containing protein 7",
  "term_id": "GO:1990756",
  "gene": "UniProtKB:Q8WVZ9"
}